{
  "term_label": "Unknown biological process",
  "gene_symbol": "BAGE5",
  "gene": "UniProtKB:Q86Y27",
  "term_id": "UNKNOWN:0002",
  "gene_name": "B melanoma antigen 5"
}